{
  "term_id": "GO:0006376",
  "gene_symbol": "LUC7L",
  "term_label": "mRNA splice site recognition",
  "gene_name": "Putative RNA-binding protein Luc7-like 1",
  "gene": "UniProtKB:Q9NQ29"
}